negative aerotaxis [GO:0052130] (biological process) Sources: GOC:dph, GOC:mtg_pamgo_17jul06 Relationships: is a type of aerotaxis [GO:0009454]; is a type of negative chemotaxis [GO:0050919]; is a type of negative energy taxis [GO:0052129] Definition: The directed movement of a motile cell or organism towards a lower concentration of environmental oxygen.